{
  "gene_name": "Zinc finger protein 143",
  "term_id": "GO:0000978",
  "term_label": "RNA polymerase II cis-regulatory region sequence-specific DNA binding",
  "gene_symbol": "ZNF143",
  "gene": "UniProtKB:P52747"
}